sucrose transmembrane transport [GO:1904982] (biological process) Relationships: is a type of sucrose transport [GO:0015770]; is a type of GO:0034219 Subtypes: GO:0106082 Definition: The process in which sucrose is transported across a membrane. References: PMID:11136464 Sources: GOC:TermGenie, GO_REF:0000069